{
  "gene_symbol": "CENPP",
  "term_label": "Unknown molecular function",
  "term_id": "UNKNOWN:0001",
  "gene": "UniProtKB:Q6IPU0",
  "gene_name": "Centromere protein P"
}